{
  "term_id": "UNKNOWN:0001",
  "term_label": "Unknown molecular function",
  "gene": "UniProtKB:Q9GZN7",
  "gene_name": "Protein rogdi homolog",
  "gene_symbol": "ROGDI"
}